regulation of unsaturated fatty acid biosynthetic process [GO:2001279] (biological process) Relationships: is a type of regulation of fatty acid biosynthetic process [GO:0042304]; regulates unsaturated fatty acid biosynthetic process [GO:0006636] Definition: Any process that modulates the frequency, rate or extent of unsaturated fatty acid biosynthetic process. Also known as: regulation of unsaturated fatty acid anabolism, regulation of unsaturated fatty acid biosynthesis, regulation of unsaturated fatty acid formation, regulation of unsaturated fatty acid synthesis, regulation of fatty acid desaturation, regulation of polyunsaturated fatty acid biosynthesis Subtypes: GO:0031392, positive regulation of unsaturated fatty acid biosynthetic process [GO:2001280] Sources: GO:0006636